{
  "term_id": "GO:0005739",
  "gene_name": "Statherin",
  "gene_symbol": "STATH",
  "gene": "UniProtKB:P02808",
  "term_label": "mitochondrion"
}